{
  "gene": "UniProtKB:Q7Z7F7",
  "term_label": "mitochondrial large ribosomal subunit",
  "gene_name": "Large ribosomal subunit protein mL55",
  "gene_symbol": "MRPL55",
  "term_id": "GO:0005762"
}